{
  "term_id": "UNKNOWN:0001",
  "term_label": "Unknown molecular function",
  "gene_name": "Uncharacterized protein",
  "gene": "UniProtKB:A0A494C0I6",
  "gene_symbol": "A0A494C0I6"
}